{
  "term_id": "GO:0000981",
  "gene_name": "Achaete-scute homolog 5",
  "gene_symbol": "ASCL5",
  "term_label": "DNA-binding transcription factor activity, RNA polymerase II-specific",
  "gene": "UniProtKB:Q7RTU5"
}